{
  "gene_symbol": "CDR2",
  "term_label": "Unknown cellular component",
  "gene_name": "Cerebellar degeneration-related protein 2",
  "gene": "UniProtKB:Q01850",
  "term_id": "UNKNOWN:0003"
}